{
  "gene_symbol": "STX12",
  "gene_name": "Syntaxin-12",
  "term_id": "GO:0008021",
  "gene": "UniProtKB:Q86Y82",
  "term_label": "synaptic vesicle"
}